positive regulation of N-terminal peptidyl-methionine acetylation [GO:1904665] (biological process) Definition: Any process that activates or increases the frequency, rate or extent of N-terminal peptidyl-methionine acetylation. References: PMID:20807799 Sources: GOC:TermGenie, GO_REF:0000058 Relationships: is a type of GO:1901985; is a type of positive regulation of protein maturation [GO:1903319]; is a type of regulation of N-terminal peptidyl-methionine acetylation [GO:1904663]; positively regulates N-terminal peptidyl-methionine acetylation [GO:0017196]